{
  "gene": "UniProtKB:O95900",
  "gene_name": "Pseudouridylate synthase TRUB2, mitochondrial",
  "term_id": "GO:0070131",
  "gene_symbol": "TRUB2",
  "term_label": "positive regulation of mitochondrial translation"
}